{
  "gene_name": "NHL repeat-containing protein 3",
  "term_label": "proteasome-mediated ubiquitin-dependent protein catabolic process",
  "gene": "UniProtKB:Q5JS37",
  "term_id": "GO:0043161",
  "gene_symbol": "NHLRC3"
}